{
  "gene_name": "Mitochondrial adenyl nucleotide antiporter SLC25A23",
  "gene": "UniProtKB:Q9BV35",
  "term_label": "ATP transmembrane transporter activity",
  "gene_symbol": "SLC25A23",
  "term_id": "GO:0005347"
}